{
  "gene": "UniProtKB:Q2I0M5",
  "gene_symbol": "RSPO4",
  "term_label": "signaling receptor binding",
  "gene_name": "R-spondin-4",
  "term_id": "GO:0005102"
}